{
  "term_id": "GO:0031982",
  "gene": "UniProtKB:Q68DD2",
  "gene_name": "Cytosolic phospholipase A2 zeta",
  "gene_symbol": "PLA2G4F",
  "term_label": "vesicle"
}